spinal cord motor neuron migration [GO:0097476] (BP) Relationships: is a type of GO:0097475 References: PMID:20711475 Sources: CL:0011001, GOC:yaf Subtypes: lateral motor column neuron migration [GO:0097477] Definition: The orderly movement of a spinal cord motor neuron from one site to another. A spinal cord motor neuron is a motor neuron that passes from the spinal cord toward or to a muscle and conducts an impulse that causes movement.